{
  "gene_symbol": "GID8",
  "term_label": "ubiquitin ligase complex",
  "gene_name": "Glucose-induced degradation protein 8 homolog",
  "term_id": "GO:0000151",
  "gene": "UniProtKB:Q9NWU2"
}